excitatory synapse assembly [GO:1904861] (biological process) Also known as: excitatory synapse formation Definition: The aggregation, arrangement and bonding together of a set of components to form an excitatory synapse. Relationships: is a type of synapse assembly [GO:0007416] Regulation: RO_0002211 by regulation of excitatory synapse assembly [GO:1904889]; negatively regulated by negative regulation of excitatory synapse assembly [GO:1904890]; positively regulated by positive regulation of excitatory synapse assembly [GO:1904891] References: PMID:21670302 Sources: GOC:PARL, GOC:TermGenie, GOC:bf, GO_REF:0000079